specification of anterior mesonephric tubule identity [GO:0072168] (BP) Definition: The process in which the tubules of the anterior mesonephros acquire their identity. Sources: GOC:mtg_kidney_jan10 Relationships: is a type of anterior/posterior pattern specification involved in kidney development [GO:0072098]; is a type of GO:0072167; is part of anterior mesonephric tubule development [GO:0072165]